regulation of biological quality [GO:0065008] (biological process) Subtypes: GO:0002026, regulation of heart rate [GO:0002027], GO:0006450, positive regulation of cytosolic calcium ion concentration [GO:0007204], GO:0008217, GO:0008360, regulation of calcium ion transport into cytosol [GO:0010522], regulation of hormone levels [GO:0010817], GO:0014729, regulation of myofibril number [GO:0014882], regulation of aggregate size involved in sorocarp development [GO:0031157], regulation of protein stability [GO:0031647], regulation of appetite [GO:0032098], regulation of muscle filament sliding speed [GO:0032972], regulation of tube architecture, open tracheal system [GO:0035152], GO:0042391, regulation of vascular permeability [GO:0043114], GO:0043487, regulation of circulating fibrinogen levels [GO:0044537], regulation of R8 cell spacing in compound eye [GO:0045468], GO:0045924, GO:0046719, regulation of synaptic plasticity [GO:0048167], GO:0050803, GO:0050878, regulation of intracellular pH [GO:0051453], GO:0051481, regulation of cilium beat frequency involved in ciliary motility [GO:0060296], regulation of protein complex stability [GO:0061635], regulation of anatomical structure size [GO:0090066], regulation of membrane permeability [GO:0090559], GO:0097035, GO:0097752, regulation of neurotransmitter receptor localization to postsynaptic specialization membrane [GO:0098696], GO:0099072, GO:0099145, regulation of postsynaptic neurotransmitter receptor internalization [GO:0099149], regulation of neurotransmitter receptor transport, endosome to postsynaptic membrane [GO:0099152], regulation of postsynaptic neurotransmitter receptor diffusion trapping [GO:0150054] Definition: Any process that modulates a qualitative or quantitative trait of a biological quality. A biological quality is a measurable attribute of an organism or part of an organism, such as size, mass, shape, color, etc. Also known as: regulation of biological attribute, regulation of biological characteristic Sources: GOC:dph, GOC:isa_complete, GOC:mah, GOC:pr, GOC:vw Relationships: is a type of biological regulation [GO:0065007]